{
  "gene": "UniProtKB:Q13733",
  "gene_symbol": "ATP1A4",
  "gene_name": "Sodium_potassium-transporting ATPase subunit alpha-4",
  "term_id": "GO:0030007",
  "term_label": "intracellular potassium ion homeostasis"
}